negative regulation of gamma-delta T cell differentiation [GO:0045587] (biological process) Note: Note that immunologists typically use the word 'development' to refer to cells of B or T cell lineages undergoing the process that GO describes as 'cell differentiation'. Also known as: down regulation of gamma-delta T cell differentiation, down-regulation of gamma-delta T cell differentiation, downregulation of gamma-delta T cell differentiation, negative regulation of gamma-delta T lymphocyte differentiation, negative regulation of gamma-delta T-cell differentiation, negative regulation of gamma-delta T-lymphocyte differentiation, inhibition of gamma-delta T cell differentiation, negative regulation of gamma-delta T cell development Relationships: is a type of negative regulation of T cell differentiation [GO:0045581]; is a type of regulation of gamma-delta T cell differentiation [GO:0045586]; is a type of negative regulation of gamma-delta T cell activation [GO:0046644]; negatively regulates gamma-delta T cell differentiation [GO:0042492] Sources: GOC:go_curators Definition: Any process that stops, prevents, or reduces the frequency, rate or extent of gamma-delta T cell differentiation.